{
  "gene_name": "Olfactory receptor 12D1",
  "gene_symbol": "OR12D1",
  "term_label": "odorant binding",
  "gene": "UniProtKB:P0DN82",
  "term_id": "GO:0005549"
}